{
  "gene_name": "Protein numb homolog",
  "gene_symbol": "NUMB",
  "gene": "UniProtKB:P49757",
  "term_id": "GO:0005737",
  "term_label": "cytoplasm"
}